response to micafungin [GO:1903967] (biological process) References: PMID:16928959 Sources: GOC:TermGenie, GO_REF:0000071 Definition: Any process that results in a change in state or activity of a cell or an organism (in terms of movement, secretion, enzyme production, gene expression, etc.) as a result of a micafungin stimulus. Subtypes: cellular response to micafungin [GO:1903968] Relationships: is a type of GO:0033993; is a type of response to nitrogen compound [GO:1901698]; is a type of GO:1901700